{
  "term_id": "UNKNOWN:0003",
  "term_label": "Unknown cellular component",
  "gene": "UniProtKB:Q9ULK2",
  "gene_name": "Ataxin-7-like protein 1",
  "gene_symbol": "ATXN7L1"
}